{
  "gene_symbol": "MAP1LC3B",
  "gene_name": "Microtubule-associated proteins 1A_1B light chain 3B",
  "term_label": "autophagosome assembly",
  "term_id": "GO:0000045",
  "gene": "UniProtKB:Q9GZQ8"
}